{
  "gene_name": "Small ubiquitin-related modifier 3",
  "term_label": "ubiquitin-like protein ligase binding",
  "term_id": "GO:0044389",
  "gene_symbol": "SUMO3",
  "gene": "UniProtKB:P55854"
}